{
  "term_id": "UNKNOWN:0001",
  "term_label": "Unknown molecular function",
  "gene": "UniProtKB:Q9NNW5",
  "gene_name": "WD repeat-containing protein 6",
  "gene_symbol": "WDR6"
}